{
  "gene_name": "Cap-specific mRNA (nucleoside-2'-O-)-methyltransferase 1",
  "term_label": "methyltransferase cap1 activity",
  "gene_symbol": "CMTR1",
  "term_id": "GO:0004483",
  "gene": "UniProtKB:Q8N1G2"
}